{
  "gene_symbol": "NEPRO",
  "gene_name": "Nucleolus and neural progenitor protein",
  "term_id": "UNKNOWN:0001",
  "term_label": "Unknown molecular function",
  "gene": "UniProtKB:Q6NW34"
}